{
  "term_label": "CXCR chemokine receptor binding",
  "gene": "UniProtKB:P02778",
  "gene_symbol": "CXCL10",
  "term_id": "GO:0045236",
  "gene_name": "C-X-C motif chemokine 10"
}